{
  "term_label": "axonemal microtubule",
  "gene": "UniProtKB:Q8N1D5",
  "term_id": "GO:0005879",
  "gene_symbol": "CFAP107",
  "gene_name": "Cilia- and flagella-associated protein 107"
}